{
  "gene": "UniProtKB:Q5NDL2",
  "term_id": "GO:0005788",
  "gene_name": "EGF domain-specific O-linked N-acetylglucosamine transferase",
  "term_label": "endoplasmic reticulum lumen",
  "gene_symbol": "EOGT"
}